{
  "term_label": "regulation of RNA splicing",
  "term_id": "GO:0043484",
  "gene": "UniProtKB:Q02040",
  "gene_symbol": "AKAP17A",
  "gene_name": "A-kinase anchor protein 17A"
}